{
  "term_id": "UNKNOWN:0001",
  "gene_symbol": "AFAP1L1",
  "gene": "UniProtKB:Q8TED9",
  "term_label": "Unknown molecular function",
  "gene_name": "Actin filament-associated protein 1-like 1"
}